{
  "term_label": "phosphatidylinositol-4,5-bisphosphate binding",
  "term_id": "GO:0005546",
  "gene_name": "GRAM domain-containing protein 2A",
  "gene": "UniProtKB:Q8IUY3",
  "gene_symbol": "GRAMD2A"
}